{
  "gene_symbol": "TRMT10C",
  "term_label": "nucleus",
  "term_id": "GO:0005634",
  "gene": "UniProtKB:Q7L0Y3",
  "gene_name": "tRNA methyltransferase 10 homolog C"
}